{
  "gene_name": "Rab3 GTPase-activating protein catalytic subunit",
  "gene": "UniProtKB:Q15042",
  "term_label": "Unknown cellular component",
  "gene_symbol": "RAB3GAP1",
  "term_id": "UNKNOWN:0003"
}